{
  "term_id": "GO:0016323",
  "gene_name": "Carbonic anhydrase-related protein 11",
  "gene_symbol": "CA11",
  "gene": "UniProtKB:O75493",
  "term_label": "basolateral plasma membrane"
}